negative regulation of terminal button organization [GO:1901613] (biological process) References: PMID:22426000 Sources: GOC:TermGenie Definition: Any process that stops, prevents or reduces the frequency, rate or extent of terminal button organization. Also known as: down regulation of bouton organization, down regulation of presynaptic bouton organization, down regulation of synaptic bouton organization, down regulation of terminal bouton organization, down regulation of terminal button organisation, down regulation of terminal button organization, down-regulation of bouton organization, down-regulation of presynaptic bouton organization, down-regulation of synaptic bouton organization, down-regulation of terminal bouton organization, down-regulation of terminal button organisation, down-regulation of terminal button organization, downregulation of bouton organization, downregulation of presynaptic bouton organization, downregulation of synaptic bouton organization, downregulation of terminal bouton organization, downregulation of terminal button organisation, downregulation of terminal button organization, negative regulation of bouton organization, negative regulation of presynaptic bouton organization, negative regulation of synaptic bouton organization, negative regulation of terminal bouton organization, negative regulation of terminal button organisation, inhibition of bouton organization, inhibition of presynaptic bouton organization, inhibition of synaptic bouton organization, inhibition of terminal bouton organization, inhibition of terminal button organisation, inhibition of terminal button organization Relationships: is a type of negative regulation of cellular component organization [GO:0051129]; is a type of regulation of terminal button organization [GO:2000331]; negatively regulates terminal button organization [GO:0072553]